1-phosphatidylinositol-4,5-bisphosphate 3-kinase activity [GO:0046934] (molecular function) Definition: Catalysis of the reaction: a 1-phosphatidyl-1D-myo-inositol 4,5-bisphosphate + ATP = a 1-phosphatidyl-1D-myo-inositol 3,4,5-trisphosphate + ADP + H+. Relationships: is a type of phosphatidylinositol kinase activity [GO:0052742] Also known as: phosphatidylinositol-4,5-bisphosphate 3-kinase activity, phosphatidylinositol 3-kinase activity, class I, phosphatidylinositol 3-kinase activity, class II, phosphatidylinositol 3-kinase, class I, catalyst activity, type I phosphoinositide 3-kinase activity Sources: EC:2.7.1.153, RHEA:21292